{
  "gene": "UniProtKB:Q9BT78",
  "term_label": "COP9 signalosome",
  "term_id": "GO:0008180",
  "gene_symbol": "COPS4",
  "gene_name": "COP9 signalosome complex subunit 4"
}